{
  "term_label": "Unknown molecular function",
  "gene_symbol": "PGRMC1",
  "gene": "UniProtKB:O00264",
  "term_id": "UNKNOWN:0001",
  "gene_name": "Membrane-associated progesterone receptor component 1"
}